extrinsic component of phagophore assembly site membrane [GO:0097632] (cellular component) Sources: GOC:mf Definition: The component of the phagophore assembly site membrane consisting of gene products and protein complexes that are loosely bound to one of its surfaces, but not integrated into the hydrophobic region. Relationships: is a type of GO:0031312; is part of phagophore assembly site membrane [GO:0034045] Also known as: extrinsic to phagophore assembly site membrane, extrinsic component of pre-autophagosomal structure membrane, phagophore assembly site peripheral membrane